{
  "gene_symbol": "LINC00518",
  "gene": "UniProtKB:Q8N0U6",
  "term_label": "Unknown cellular component",
  "gene_name": "Putative uncharacterized protein encoded by LINC00518",
  "term_id": "UNKNOWN:0003"
}